cellular response to borneol [GO:1905231] (biological process) Relationships: is a type of cellular response to lipid [GO:0071396]; is a type of response to borneol [GO:1905230] References: PMID:26593909 Sources: GOC:TermGenie, GO_REF:0000071 Definition: Any process that results in a change in state or activity of a cell (in terms of movement, secretion, enzyme production, gene expression, etc.) as a result of a borneol stimulus.